symbiont-mediated perturbation of host cholinergic synaptic transmission [GO:0044760] (biological process) Sources: GOC:jl Relationships: is a type of symbiont-mediated perturbation of host synaptic transmission [GO:0044758] Definition: A process in which a symbiont alters or subverts cholinergic synaptic transmission, the communication from a neuron to a target (neuron, muscle, or secretory cell) across a synapse via the neurotransmitter choline, in its host organism. Subtypes: GO:0044761 Also known as: modulation by symbiont of host cholinergic synaptic transmission, regulation by symbiont of host cholinergic synaptic transmission